{
  "gene": "UniProtKB:Q7Z4H8",
  "gene_symbol": "POGLUT3",
  "term_label": "endomembrane system",
  "gene_name": "Protein O-glucosyltransferase 3",
  "term_id": "GO:0012505"
}